{
  "term_label": "action potential",
  "gene_symbol": "KCNC1",
  "gene_name": "Potassium voltage-gated channel subfamily C member 1",
  "term_id": "GO:0001508",
  "gene": "UniProtKB:P48547"
}